has_obo_format_version [oboInOwl#hasOBOFormatVersion]